{
  "term_id": "GO:0005634",
  "gene_name": "Multifunctional methyltransferase subunit TRM112-like protein",
  "gene_symbol": "TRMT112",
  "term_label": "nucleus",
  "gene": "UniProtKB:Q9UI30"
}